activin AB complex [GO:0048183] (cellular component) Definition: A nonsteroidal regulator, composed of two covalently linked inhibin beta subunits (sometimes known as activin beta or activin/inhibin beta), inhibin beta-A and inhibin beta-B. Sources: GOC:go_curators Also known as: inhibin beta-A, inhibin beta-B Note: Note that the actions of the activin complex are the opposite of those of the inhibin complex, which is a dimer of an inhibin beta-A or inhibin beta-B subunit and a inhibin alpha subunit. See 'inhibin complex ; GO:0043511'. Relationships: is a type of activin complex [GO:0048180]